{
  "term_label": "Unknown biological process",
  "gene": "UniProtKB:A0A0A6YYL3",
  "gene_name": "POTE ankyrin domain family member B",
  "term_id": "UNKNOWN:0002",
  "gene_symbol": "POTEB"
}